regulation of ascospore wall beta-glucan biosynthetic process [GO:0060622] (biological process) Relationships: is a type of regulation of cell cycle process [GO:0010564]; is a type of regulation of fungal-type cell wall beta-glucan biosynthetic process [GO:0090093]; is a type of regulation of reproductive process [GO:2000241]; regulates GO:0034412 Definition: Any process that modulates the rate, frequency or extent of ascospore wall beta-glucan biosynthetic process, the chemical reactions and pathways resulting in the formation of beta-glucans, compounds composed of glucose residues linked by beta-D-glucosidic bonds, found in the walls of ascospores. Subtypes: GO:0060624 Sources: GOC:dph, GOC:tb